{
  "term_id": "GO:0031982",
  "gene_name": "Alpha-1,3-galactosyltransferase 2",
  "term_label": "vesicle",
  "gene": "UniProtKB:U3KPV4",
  "gene_symbol": "A3GALT2"
}